{
  "term_label": "Unknown biological process",
  "gene": "UniProtKB:Q9NS18",
  "gene_symbol": "GLRX2",
  "gene_name": "Glutaredoxin-2, mitochondrial",
  "term_id": "UNKNOWN:0002"
}